{
  "term_id": "GO:0043325",
  "gene_symbol": "HIP1",
  "gene_name": "Huntingtin-interacting protein 1",
  "gene": "UniProtKB:O00291",
  "term_label": "phosphatidylinositol-3,4-bisphosphate binding"
}